{
  "term_id": "GO:0030139",
  "gene": "UniProtKB:Q8TEU7",
  "term_label": "endocytic vesicle",
  "gene_symbol": "RAPGEF6",
  "gene_name": "Rap guanine nucleotide exchange factor 6"
}